protein kinase A regulatory subunit binding [GO:0034237] (molecular function) Relationships: is a type of GO:0051018 Definition: Binding to one or both of the regulatory subunits of protein kinase A. Also known as: PKA regulatory subunit binding, protein kinase A anchoring activity Sources: GOC:mah